{
  "term_label": "nucleus",
  "term_id": "GO:0005634",
  "gene": "UniProtKB:Q86V20",
  "gene_name": "Shieldin complex subunit 2",
  "gene_symbol": "SHLD2"
}